{
  "term_id": "GO:0016477",
  "gene": "UniProtKB:Q9Y6N8",
  "gene_symbol": "CDH10",
  "term_label": "cell migration",
  "gene_name": "Cadherin-10"
}